{
  "term_id": "GO:0007224",
  "gene_name": "Transcriptional activator GLI3",
  "gene_symbol": "GLI3",
  "gene": "UniProtKB:P10071",
  "term_label": "smoothened signaling pathway"
}